regulation of Purkinje myocyte action potential [GO:0098906] (biological process) Relationships: is_a regulation of cell communication [GO:0010646]; is a type of regulation of cardiac muscle cell action potential [GO:0098901]; regulates Purkinje myocyte action potential [GO:0086017] Sources: GOC:BHF, GOC:mtg_cardiac_conduct_nov11 Definition: Any process that modulates the frequency, rate or extent of action potential creation, propagation or termination in a Purkinje myocyte. This typically occurs via modulation of the activity or expression of voltage-gated ion channels.